response to triglyceride [GO:0034014] (biological process) Subtypes: cellular response to triglyceride [GO:0071401] Sources: GOC:sl Definition: Any process that results in a change in state or activity of a cell or an organism (in terms of movement, secretion, enzyme production, gene expression, etc.) as a result of a triglyceride stimulus. Relationships: is a type of response to lipid [GO:0033993]; is_a GO:1901700 Also known as: response to triacylglyceride, response to triacylglycerol